{
  "term_id": "GO:0046471",
  "gene_symbol": "PLA2G2E",
  "gene": "UniProtKB:Q9NZK7",
  "gene_name": "Group IIE secretory phospholipase A2",
  "term_label": "phosphatidylglycerol metabolic process"
}